{
  "gene_symbol": "ZSCAN25",
  "term_id": "UNKNOWN:0003",
  "gene_name": "Zinc finger and SCAN domain-containing protein 25",
  "term_label": "Unknown cellular component",
  "gene": "UniProtKB:Q6NSZ9"
}